{
  "gene_symbol": "FGF23",
  "gene": "UniProtKB:Q9GZV9",
  "term_label": "positive regulation of cell population proliferation",
  "term_id": "GO:0008284",
  "gene_name": "Fibroblast growth factor 23"
}